zf-TRAF domain binding [GO:0044198] (molecular function) Also known as: TRAF-type zinc finger domain binding, zinc finger TRAF-type domain binding, zinc-finger-TRAF domain binding Definition: Binding to a TRAF-type zinc finger domain of a protein. Relationships: is a type of GO:0019904 Sources: InterPro:IPR001293